{
  "gene_symbol": "CEACAM7",
  "term_id": "GO:0009986",
  "gene_name": "Carcinoembryonic antigen-related cell adhesion molecule 7",
  "term_label": "cell surface",
  "gene": "UniProtKB:Q14002"
}